{
  "gene_symbol": "CAMSAP3",
  "gene": "UniProtKB:Q9P1Y5",
  "term_id": "GO:0043111",
  "gene_name": "Calmodulin-regulated spectrin-associated protein 3",
  "term_label": "replication fork arrest"
}